{
  "term_id": "GO:0036038",
  "gene": "UniProtKB:Q96GX1",
  "gene_symbol": "TCTN2",
  "term_label": "MKS complex",
  "gene_name": "Tectonic-2"
}